{
  "term_label": "DNA-binding transcription factor activity, RNA polymerase II-specific",
  "gene_symbol": "LHX6",
  "term_id": "GO:0000981",
  "gene_name": "LIM_homeobox protein Lhx6",
  "gene": "UniProtKB:Q9UPM6"
}